{
  "gene_symbol": "NPIPA2",
  "gene": "UniProtKB:E9PIF3",
  "gene_name": "Nuclear pore complex-interacting protein family member A2",
  "term_id": "UNKNOWN:0003",
  "term_label": "Unknown cellular component"
}